{
  "gene_symbol": "C1QBP",
  "term_id": "GO:0003714",
  "gene": "UniProtKB:Q07021",
  "term_label": "transcription corepressor activity",
  "gene_name": "Complement component 1 Q subcomponent-binding protein, mitochondrial"
}